{
  "gene_name": "Inhibin beta C chain",
  "gene": "UniProtKB:P55103",
  "term_id": "GO:0005615",
  "gene_symbol": "INHBC",
  "term_label": "extracellular space"
}